{
  "gene": "UniProtKB:Q96F85",
  "gene_symbol": "CNRIP1",
  "gene_name": "CB1 cannabinoid receptor-interacting protein 1",
  "term_id": "GO:0031718",
  "term_label": "type 1 cannabinoid receptor binding"
}